{
  "term_id": "GO:0003924",
  "gene": "UniProtKB:Q5VTM2",
  "gene_name": "Arf-GAP with GTPase, ANK repeat and PH domain-containing protein 9",
  "term_label": "GTPase activity",
  "gene_symbol": "AGAP9"
}